alpha-pinene monooxygenase (NADH) activity [GO:0018634] (molecular function) Definition: Catalysis of the reaction: alpha-pinene + NADH + H+ + O2 = NAD+ + H2O + alpha-pinene oxide. Relationships: is a type of oxidoreductase activity, acting on paired donors, with incorporation or reduction of molecular oxygen, NAD(P)H as one donor, and incorporation of one atom of oxygen [GO:0016709] Sources: RHEA:32891 Also known as: alpha-pinene monooxygenase [NADH] activity